{
  "term_id": "GO:0043065",
  "gene_name": "Serine_threonine-protein kinase LATS2",
  "gene": "UniProtKB:Q9NRM7",
  "gene_symbol": "LATS2",
  "term_label": "positive regulation of apoptotic process"
}